{
  "gene_symbol": "SGK3",
  "gene_name": "Serine_threonine-protein kinase Sgk3",
  "term_id": "GO:0015459",
  "term_label": "potassium channel regulator activity",
  "gene": "UniProtKB:Q96BR1"
}